caveola [GO:0005901] (cellular component) Definition: A membrane raft that forms small pit, depression, or invagination that communicates with the outside of a cell and extends inward, indenting the cytoplasm and the cell membrane. Examples include flask-shaped invaginations of the plasma membrane in adipocytes associated with caveolin proteins, and minute pits or incuppings of the cell membrane formed during pinocytosis. Caveolae may be pinched off to form free vesicles within the cytoplasm. References: PMID:16645198 Sources: GOC:mah, ISBN:0721662544 Relationships: is a type of plasma membrane raft [GO:0044853] Also known as: caveolae, caveolar membrane